{
  "term_label": "Unknown biological process",
  "term_id": "UNKNOWN:0002",
  "gene": "UniProtKB:Q9UBW8",
  "gene_name": "COP9 signalosome complex subunit 7a",
  "gene_symbol": "COPS7A"
}